{
  "gene_name": "Zinc finger protein ZFPM2",
  "gene": "UniProtKB:Q8WW38",
  "gene_symbol": "ZFPM2",
  "term_label": "heart development",
  "term_id": "GO:0007507"
}